{
  "gene_symbol": "ANKS1A",
  "gene_name": "Ankyrin repeat and SAM domain-containing protein 1A",
  "gene": "UniProtKB:Q92625",
  "term_label": "cytosol",
  "term_id": "GO:0005829"
}